{
  "gene_symbol": "GFPT2",
  "gene_name": "Glutamine--fructose-6-phosphate aminotransferase [isomerizing] 2",
  "term_label": "fructose 6-phosphate metabolic process",
  "gene": "UniProtKB:O94808",
  "term_id": "GO:0006002"
}